{
  "term_label": "Unknown biological process",
  "gene_name": "Protein FAM193A",
  "gene_symbol": "FAM193A",
  "term_id": "UNKNOWN:0002",
  "gene": "UniProtKB:P78312"
}